{
  "gene_symbol": "CHMP4B",
  "term_id": "GO:0005771",
  "term_label": "multivesicular body",
  "gene_name": "Charged multivesicular body protein 4b",
  "gene": "UniProtKB:Q9H444"
}